mesenchyme development [GO:0060485] (biological process) Subtypes: endocardial cushion development [GO:0003197], GO:0003342, GO:0003343, gonadal mesoderm development [GO:0007506], GO:0048339, lateral mesoderm development [GO:0048368], GO:0060484, GO:0061056, kidney mesenchyme development [GO:0072074], metanephric cortex development [GO:0072214] Also known as: mesenchymal development Relationships: is a type of GO:0009888; is part of animal organ development [GO:0048513] Sources: GOC:dph Definition: The process whose specific outcome is the progression of a mesenchymal tissue over time, from its formation to the mature structure. A mesenchymal tissue is made up of loosely packed stellate cells.